salicylic acid biosynthetic process [GO:0009697] (BP) Regulation: regulated by regulation of salicylic acid biosynthetic process [GO:0080142] Relationships: is_a salicylic acid metabolic process [GO:0009696]; is a type of phenol-containing compound biosynthetic process [GO:0046189]; is a type of monocarboxylic acid biosynthetic process [GO:0072330] Definition: The chemical reactions and pathways resulting in the formation of salicylic acid (2-hydroxybenzoic acid), a derivative of benzoic acid. Sources: ISBN:0943088399 Also known as: salicylate biosynthetic process, salicylic acid anabolism, salicylic acid biosynthesis, salicylic acid formation, salicylic acid synthesis